{
  "gene": "UniProtKB:B2CW77",
  "term_label": "Unknown biological process",
  "gene_name": "Killin",
  "gene_symbol": "KLLN",
  "term_id": "UNKNOWN:0002"
}